regulation of photomorphogenesis [GO:0010099] (biological process) Sources: GOC:tb Subtypes: negative regulation of photomorphogenesis [GO:0010100], GO:2000306 Relationships: is a type of regulation of post-embryonic development [GO:0048580]; is a type of GO:2000030; regulates photomorphogenesis [GO:0009640] Definition: Any process that modulates the rate or extent of photomorphogenesis.